{
  "gene_symbol": "MYBBP1A",
  "term_label": "sequence-specific DNA binding",
  "term_id": "GO:0043565",
  "gene": "UniProtKB:Q9BQG0",
  "gene_name": "Myb-binding protein 1A"
}